{
  "gene_name": "Thioredoxin domain-containing protein 6",
  "term_label": "Unknown cellular component",
  "term_id": "UNKNOWN:0003",
  "gene": "UniProtKB:Q86XW9",
  "gene_symbol": "NME9"
}